Cdc24p-Far1p-Gbetagamma complex [GO:0120171] (cellular component) References: PMID:10087263 Definition: A complex that forms at the cell cortex in response to pheromone treatment and is required for the polarized growth of haploid yeast cells towards a mating partner during yeast mating. In the yeast Saccharomyces cerevisiae, this complex consists of Cdc24p, Far1p, Ste4p (G-protein beta subunit) and Ste18p (G-protein gamma subunit). Also known as: CDC24-FAR1-BG complex, CDC24-FAR1-Gbetagamma complex, Cdc24p-Far1p-BG complex Relationships: is a type of GO:0032991